{
  "term_label": "DNA-binding transcription factor activity, RNA polymerase II-specific",
  "term_id": "GO:0000981",
  "gene": "UniProtKB:P35680",
  "gene_symbol": "HNF1B",
  "gene_name": "Hepatocyte nuclear factor 1-beta"
}